{
  "term_id": "GO:0061630",
  "term_label": "ubiquitin protein ligase activity",
  "gene_name": "Tripartite motif-containing protein 2",
  "gene_symbol": "TRIM2",
  "gene": "UniProtKB:Q9C040"
}